intermediate filament cytoskeleton organization [GO:0045104] (biological process) Also known as: intermediate filament cytoskeleton organisation, intermediate filament cytoskeleton organization and biogenesis Definition: A process that is carried out at the cellular level which results in the assembly, arrangement of constituent parts, or disassembly of cytoskeletal structures comprising intermediate filaments and their associated proteins. Sources: GOC:ai Relationships: is_a cytoskeleton organization [GO:0007010]; is a type of intermediate filament-based process [GO:0045103] Subtypes: GO:0045109, neurofilament cytoskeleton organization [GO:0060052], postsynaptic intermediate filament cytoskeleton organization [GO:0099185]